{
  "gene": "UniProtKB:Q5HYK7",
  "term_id": "GO:0005886",
  "gene_name": "SH3 domain-containing protein 19",
  "gene_symbol": "SH3D19",
  "term_label": "plasma membrane"
}